{
  "gene_name": "Transmembrane protein 145",
  "term_id": "UNKNOWN:0003",
  "gene": "UniProtKB:Q8NBT3",
  "term_label": "Unknown cellular component",
  "gene_symbol": "TMEM145"
}